{
  "gene_name": "Thymosin beta 15B",
  "gene": "UniProtKB:A0A087X1C1",
  "term_id": "UNKNOWN:0001",
  "term_label": "Unknown molecular function",
  "gene_symbol": "TMSB15B"
}